{
  "term_label": "Unknown molecular function",
  "gene_symbol": "FAM186A",
  "term_id": "UNKNOWN:0001",
  "gene": "UniProtKB:A6NE01",
  "gene_name": "Protein FAM186A"
}